{
  "gene_symbol": "CD44",
  "term_id": "GO:0070374",
  "term_label": "positive regulation of ERK1 and ERK2 cascade",
  "gene": "UniProtKB:P16070",
  "gene_name": "CD44 antigen"
}